dicarboxylic acid metabolic process [GO:0043648] (biological process) Sources: ISBN:0198506732 Also known as: dicarboxylate metabolic process, dicarboxylate metabolism, dicarboxylic acid metabolism Subtypes: 2-oxoglutarate metabolic process [GO:0006103], succinate metabolic process [GO:0006105], GO:0006106, oxaloacetate metabolic process [GO:0006107], malate metabolic process [GO:0006108], GO:0006531, GO:0006536, 10-formyltetrahydrofolate metabolic process [GO:0009256], GO:0019580, protocatechuate catabolic process, ortho-cleavage [GO:0019618], oxalate metabolic process [GO:0033609], D-glucarate metabolic process [GO:0042836], dicarboxylic acid catabolic process [GO:0043649], dicarboxylic acid biosynthetic process [GO:0043650], chorismate metabolic process [GO:0046417], dihydrofolate metabolic process [GO:0046452], folic acid metabolic process [GO:0046655], quinolinate metabolic process [GO:0046874] Relationships: is a type of carboxylic acid metabolic process [GO:0019752] Definition: The chemical reactions and pathways involving dicarboxylic acids, any organic acid containing two carboxyl (COOH) groups or anions (COO-).